{
  "gene_name": "Solute carrier family 41 member 1",
  "term_label": "Unknown biological process",
  "term_id": "UNKNOWN:0002",
  "gene": "UniProtKB:Q8IVJ1",
  "gene_symbol": "SLC41A1"
}